{
  "term_id": "GO:0019799",
  "term_label": "tubulin N-acetyltransferase activity",
  "gene_name": "Alpha-tubulin N-acetyltransferase 1",
  "gene": "UniProtKB:Q5SQI0",
  "gene_symbol": "ATAT1"
}